{
  "term_id": "GO:0016035",
  "term_label": "zeta DNA polymerase complex",
  "gene": "UniProtKB:O60673",
  "gene_symbol": "REV3L",
  "gene_name": "DNA polymerase zeta catalytic subunit"
}